{
  "term_label": "Unknown molecular function",
  "term_id": "UNKNOWN:0001",
  "gene_name": "Protein CREG2",
  "gene": "UniProtKB:Q8IUH2",
  "gene_symbol": "CREG2"
}